{
  "term_id": "GO:0005759",
  "term_label": "mitochondrial matrix",
  "gene": "UniProtKB:Q9H6R3",
  "gene_name": "Acyl-CoA synthetase short-chain family member 3, mitochondrial",
  "gene_symbol": "ACSS3"
}